{
  "gene_symbol": "ELANE",
  "gene_name": "Neutrophil elastase",
  "term_label": "serine-type endopeptidase activity",
  "gene": "UniProtKB:P08246",
  "term_id": "GO:0004252"
}